{
  "gene_name": "Fibroblast growth factor 6",
  "gene_symbol": "FGF6",
  "gene": "UniProtKB:P10767",
  "term_id": "GO:0043410",
  "term_label": "positive regulation of MAPK cascade"
}